detection of bacterial lipopeptide [GO:0070340] (biological process) Definition: The series of events in which a bacterial lipopeptide stimulus is received by a cell and converted into a molecular signal. References: PMID:12077222 Sources: GOC:add Relationships: is a type of detection of bacterial lipoprotein [GO:0042494]; is a type of response to bacterial lipopeptide [GO:0070339] Subtypes: detection of triacyl bacterial lipopeptide [GO:0042495], detection of diacyl bacterial lipopeptide [GO:0042496]